heat dissipation [GO:0031653] (biological process) Definition: Any homeostatic process in which an organism releases excess heat to the environment, thereby lowering its internal temperature. Relationships: is a type of GO:0001659 Sources: GOC:mah Regulation: regulated by regulation of heat dissipation [GO:0031654]; negatively regulated by negative regulation of heat dissipation [GO:0031655]; positively regulated by positive regulation of heat dissipation [GO:0031656]